{
  "term_id": "GO:0006401",
  "gene_symbol": "RNASEH2C",
  "gene_name": "Ribonuclease H2 subunit C",
  "term_label": "RNA catabolic process",
  "gene": "UniProtKB:Q8TDP1"
}